response to sodium phosphate [GO:1904383] (biological process) Subtypes: GO:1904384 Relationships: is a type of GO:1902074 References: PMID:24625659 Sources: GOC:TermGenie, GO_REF:0000071 Definition: Any process that results in a change in state or activity of a cell or an organism (in terms of movement, secretion, enzyme production, gene expression, etc.) as a result of a sodium phosphate stimulus.